{
  "gene_name": "Kynureninase",
  "term_id": "GO:0019441",
  "gene": "UniProtKB:Q16719",
  "gene_symbol": "KYNU",
  "term_label": "L-tryptophan catabolic process to kynurenine"
}